myeloid dendritic cell chemotaxis [GO:0002408] (biological process) Definition: The movement of a myeloid dendritic cell in response to an external stimulus. Relationships: is a type of dendritic cell chemotaxis [GO:0002407]; is a type of myeloid leukocyte migration [GO:0097529] References: PMID:15814331, PMID:16056255 Sources: GOC:add, ISBN:0781735149 Subtypes: Langerhans cell chemotaxis [GO:0002409] Regulation: RO_0002211 by regulation of myeloid dendritic cell chemotaxis [GO:2000527]; negatively regulated by negative regulation of myeloid dendritic cell chemotaxis [GO:2000528]; positively regulated by GO:2000529